positive regulation of miRNA metabolic process [GO:2000630] (biological process) Also known as: positive regulation of microRNA metabolic process Relationships: is a type of positive regulation of RNA metabolic process [GO:0051254]; is a type of regulation of miRNA metabolic process [GO:2000628]; positively regulates miRNA metabolic process [GO:0010586] Subtypes: positive regulation of miRNA transcription [GO:1902895], GO:2000627 Definition: Any process that activates or increases the frequency, rate or extent of miRNA metabolic process. Sources: GOC:dph